{
  "gene": "UniProtKB:Q17R89",
  "term_id": "GO:0035021",
  "term_label": "negative regulation of Rac protein signal transduction",
  "gene_symbol": "ARHGAP44",
  "gene_name": "Rho GTPase-activating protein 44"
}